pyrimidine-5'-nucleotide nucleosidase activity [GO:0047405] (molecular function) Sources: EC:3.2.2.10, MetaCyc:3.2.2.10-RXN Also known as: Pyr5N activity, pyrimidine nucleotide N-ribosidase activity, pyrimidine-5'-nucleotide phosphoribo(deoxyribo)hydrolase activity Definition: Catalysis of the reaction: H2O + a pyrimidine 5'-nucleotide = ribose-5-phosphate + a pyrimidine. Relationships: is a type of hydrolase activity, hydrolyzing N-glycosyl compounds [GO:0016799]